{
  "term_label": "extracellular space",
  "gene_symbol": "C1QL3",
  "term_id": "GO:0005615",
  "gene": "UniProtKB:Q5VWW1",
  "gene_name": "Complement C1q-like protein 3"
}